alpha-N-acetylneuraminyl-2,3-beta-galactosyl-1,3-N-acetyl-galactosaminide 6-alpha-sialyltransferase activity [GO:0047290] (molecular function) Sources: RHEA:53896 Also known as: (alpha-N-acetylneuraminyl-2,3-beta-galactosyl-1,3)-N-acetylgalactosaminide alpha-2,6-sialyltransferase activity, NeuAc-alpha-2,3-Gal-beta-1,3-GalNAc-alpha-2,6-sialyltransferase activity, ST6GALNAC activity, alpha-N-acetylneuraminyl-2,3-beta-galactosyl-1,3-N-acetyl-galactosaminide alpha-2,6-sialyltransferase activity, cytidine monophosphoacetylneuraminate-(alpha-N-acetylneuraminyl-2,3-beta-galactosyl-1,3)-N-acetylgalactosaminide-alpha-2,6-sialyltransferase activity, sialyltransferase activity Definition: Catalysis of the reaction: alpha-N-acetylneuraminyl-(2->3)-beta-D-galactosyl-(1->3)-N-acetyl-D-galactosaminyl-R + CMP-N-acetyl-beta-neuraminate = alpha-N-acetylneuraminyl-(2->3)-beta-D-galactosyl-(1->3)-[N-acetyl-alpha-neuraminyl-(2->6)]-N-acetyl-D-galactosaminyl-R + CMP. Relationships: is a type of GO:0008373